lactose catabolic process, using glucoside 3-dehydrogenase [GO:0019513] (biological process) Relationships: is a type of GO:0005990; has part glucoside 3-dehydrogenase activity [GO:0033757] Sources: GOC:jl Also known as: lactose breakdown, using glucoside 3-dehydrogenase, lactose degradation, using glucoside 3-dehydrogenase Definition: The chemical reactions and pathways resulting in the breakdown of lactose, catalyzed by the enzyme glucoside 3-dehydrogenase.